diacylglycerol metabolic process [GO:0046339] (biological process) References: PMID:11481335 Relationships: is a type of acylglycerol metabolic process [GO:0006639] Subtypes: diacylglycerol biosynthetic process [GO:0006651], GO:0036154, diacylglycerol catabolic process [GO:0046340] Definition: The chemical reactions and pathways involving diacylglycerol, a glyceride in which any two of the R groups (positions not specified) are acyl groups while the remaining R group can be either H or an alkyl group. Also known as: diacylglycerol metabolism, diglyceride metabolism